{
  "gene_name": "E3 ubiquitin-protein ligase RNF138",
  "term_id": "GO:0003697",
  "gene_symbol": "RNF138",
  "gene": "UniProtKB:Q8WVD3",
  "term_label": "single-stranded DNA binding"
}